iodophenol O-methyltransferase activity [GO:0030737] (molecular function) Sources: EC:2.1.1.26, RHEA:14313 Relationships: is a type of GO:0008757 Definition: Catalysis of the reaction: 2-iodophenol + S-adenosyl-L-methionine = 1-iodo-2-methoxybenzene + S-adenosyl-L-homocysteine + H+. Also known as: S-adenosyl-L-methionine:2-iodophenol O-methyltransferase activity